{
  "term_label": "Unknown molecular function",
  "gene": "UniProtKB:A6NMD2",
  "gene_symbol": "GOLGA8J",
  "gene_name": "Golgin subfamily A member 8J",
  "term_id": "UNKNOWN:0001"
}